{
  "term_label": "ribonucleoprotein complex",
  "gene_name": "CUGBP Elav-like family member 5",
  "term_id": "GO:1990904",
  "gene_symbol": "CELF5",
  "gene": "UniProtKB:Q8N6W0"
}